creatine metabolic process [GO:0006600] (biological process) Definition: The chemical reactions and pathways involving creatine (N-(aminoiminomethyl)-N-methylglycine), a compound synthesized from the amino acids arginine, glycine, and methionine that occurs in muscle. Sources: GOC:jl, ISBN:0192801023 Also known as: creatine metabolism Subtypes: creatine biosynthetic process [GO:0006601] Relationships: is a type of modified amino acid metabolic process [GO:0006575]; is a type of GO:0032787